{
  "gene_symbol": "P4HA3",
  "gene_name": "Prolyl 4-hydroxylase subunit alpha-3",
  "gene": "UniProtKB:Q7Z4N8",
  "term_label": "endoplasmic reticulum",
  "term_id": "GO:0005783"
}